low-density lipoprotein particle disassembly involved in cholesterol transport [GO:0090121] (biological process) Sources: GOC:ascb_2009, GOC:dph, GOC:tb Relationships: is_a low-density lipoprotein particle disassembly [GO:0090495]; is part of cholesterol transport [GO:0030301] Definition: The disassembly into constituent parts of the low-density lipoprotein particle in the lysosome that contributes to cholesterol transport.